{
  "gene_name": "Olfactory receptor 5B21",
  "term_id": "GO:0007608",
  "gene": "UniProtKB:A6NL26",
  "gene_symbol": "OR5B21",
  "term_label": "sensory perception of smell"
}